{
  "gene_symbol": "CORO1C",
  "gene_name": "Coronin-1C",
  "term_label": "plasma membrane",
  "term_id": "GO:0005886",
  "gene": "UniProtKB:Q9ULV4"
}